{
  "gene_name": "ELKS_Rab6-interacting_CAST family member 1",
  "term_label": "structural constituent of presynaptic active zone",
  "term_id": "GO:0098882",
  "gene_symbol": "ERC1",
  "gene": "UniProtKB:Q8IUD2"
}